{
  "term_label": "glycine import into mitochondrion",
  "gene_name": "Mitochondrial glycine transporter",
  "term_id": "GO:1904983",
  "gene": "UniProtKB:Q96DW6",
  "gene_symbol": "SLC25A38"
}